{
  "term_id": "UNKNOWN:0003",
  "gene": "UniProtKB:Q96LR9",
  "gene_symbol": "APOLD1",
  "gene_name": "Apolipoprotein L domain-containing protein 1",
  "term_label": "Unknown cellular component"
}